{
  "term_id": "GO:0035725",
  "gene_symbol": "SLC6A18",
  "gene_name": "Inactive sodium-dependent neutral amino acid transporter B(0)AT3",
  "gene": "UniProtKB:Q96N87",
  "term_label": "sodium ion transmembrane transport"
}